regulation of protein localization to cell leading edge [GO:1905871] (biological process) Relationships: is a type of regulation of protein localization [GO:0032880]; regulates protein localization to cell leading edge [GO:1902463] Subtypes: GO:1905872, positive regulation of protein localization to cell leading edge [GO:1905873] Definition: Any process that modulates the frequency, rate or extent of protein localization to cell leading edge. References: PMID:26324884 Sources: GOC:TermGenie, GO_REF:0000058 Also known as: regulation of protein localisation in cell leading edge, regulation of protein localisation to cell leading edge, regulation of protein localization in cell leading edge